{
  "gene_name": "Fin bud initiation factor homolog",
  "gene_symbol": "FIBIN",
  "term_id": "UNKNOWN:0002",
  "gene": "UniProtKB:Q8TAL6",
  "term_label": "Unknown biological process"
}